{
  "gene": "UniProtKB:P18509",
  "term_id": "GO:0051428",
  "gene_symbol": "ADCYAP1",
  "gene_name": "Pituitary adenylate cyclase-activating polypeptide",
  "term_label": "peptide hormone receptor binding"
}